{
  "gene": "UniProtKB:Q16352",
  "gene_name": "Alpha-internexin",
  "term_id": "GO:0099184",
  "term_label": "structural constituent of postsynaptic intermediate filament cytoskeleton",
  "gene_symbol": "INA"
}